{
  "term_id": "GO:0043843",
  "gene_symbol": "ADPGK",
  "term_label": "ADP-specific glucokinase activity",
  "gene_name": "ADP-dependent glucokinase",
  "gene": "UniProtKB:Q9BRR6"
}